positive regulation of retrograde trans-synaptic signaling by neuropeptide [GO:1905434] (biological process) Relationships: is a type of positive regulation of cell communication [GO:0010647]; is a type of GO:0023056; is a type of GO:1905432; positively regulates retrograde trans-synaptic signaling by neuropeptide [GO:0099082] Definition: Any process that activates or increases the frequency, rate or extent of retrograde trans-synaptic signaling by neuropeptide. References: PMID:19448629 Sources: GOC:PARL, GOC:TermGenie, GOC:bf, GO_REF:0000058 Also known as: up regulation of retrograde trans-synaptic signaling by neuropeptide, up-regulation of retrograde trans-synaptic signaling by neuropeptide, upregulation of retrograde trans-synaptic signaling by neuropeptide, activation of retrograde trans-synaptic signaling by neuropeptide, positive regulation of neuropeptide-mediated retrograde trans-synaptic signaling